{
  "gene": "UniProtKB:Q9P1Y6",
  "term_id": "UNKNOWN:0002",
  "gene_symbol": "PHRF1",
  "gene_name": "PHD and RING finger domain-containing protein 1",
  "term_label": "Unknown biological process"
}